{
  "term_id": "UNKNOWN:0002",
  "gene_symbol": "SLC25A11",
  "gene_name": "Mitochondrial 2-oxoglutarate_malate carrier protein",
  "gene": "UniProtKB:Q02978",
  "term_label": "Unknown biological process"
}